{
  "term_id": "GO:0008360",
  "gene_symbol": "CDC42EP2",
  "gene": "UniProtKB:O14613",
  "gene_name": "Cdc42 effector protein 2",
  "term_label": "regulation of cell shape"
}